{
  "term_label": "extracellular matrix structural constituent conferring tensile strength",
  "gene": "UniProtKB:Q14031",
  "term_id": "GO:0030020",
  "gene_symbol": "COL4A6",
  "gene_name": "Collagen alpha-6(IV) chain"
}